{
  "gene": "UniProtKB:O14493",
  "gene_symbol": "CLDN4",
  "gene_name": "Claudin-4",
  "term_label": "plasma membrane",
  "term_id": "GO:0005886"
}